{
  "gene_name": "A disintegrin and metalloproteinase with thrombospondin motifs 2",
  "term_label": "extracellular matrix",
  "gene_symbol": "ADAMTS2",
  "term_id": "GO:0031012",
  "gene": "UniProtKB:O95450"
}